{
  "gene_symbol": "HNRNPUL2",
  "term_id": "GO:0003723",
  "gene_name": "Heterogeneous nuclear ribonucleoprotein U-like protein 2",
  "gene": "UniProtKB:Q1KMD3",
  "term_label": "RNA binding"
}